{
  "gene": "UniProtKB:P25940",
  "term_id": "GO:0030020",
  "gene_symbol": "COL5A3",
  "term_label": "extracellular matrix structural constituent conferring tensile strength",
  "gene_name": "Collagen alpha-3(V) chain"
}